{
  "gene_name": "ATP-dependent DNA helicase Q1",
  "gene": "UniProtKB:P46063",
  "gene_symbol": "RECQL",
  "term_label": "four-way junction helicase activity",
  "term_id": "GO:0009378"
}